positive regulation of sporangiospore formation [GO:0075287] (biological process) Subtypes: positive regulation of zoospore formation [GO:0075241], positive regulation of aplanospore formation [GO:0075291] Relationships: is a type of GO:0043945; is a type of GO:0075286; positively regulates sporangiospore formation [GO:0034300] Sources: GOC:pamgo_curators Definition: Any process that activates, maintains or increases the frequency, rate or extent of sporangiospore formation, a process in which sporangiospores, a type of asexual spore found in fungi, are formed. Sporangiospores are formed within sac-like structure, the sporangium, following the division of the cytoplasm.